{
  "term_label": "Unknown biological process",
  "term_id": "UNKNOWN:0002",
  "gene_symbol": "MON1B",
  "gene": "UniProtKB:Q7L1V2",
  "gene_name": "Vacuolar fusion protein MON1 homolog B"
}